{
  "gene_name": "Protein FAM3C",
  "term_id": "GO:0005125",
  "gene": "UniProtKB:Q92520",
  "gene_symbol": "FAM3C",
  "term_label": "cytokine activity"
}